dendritic cell dendrite assembly [GO:0097026] (biological process) Definition: Formation of dendrites, branched cellular projections (or cytoplasmic extension) that are extended from the surface of a dendritic immune cell, and which enable the cell to sample luminal pathogens and increase the surface area for antigen presentation to T cells. Also known as: dendritic extension Relationships: is a type of plasma membrane bounded cell projection assembly [GO:0120031] Regulation: regulated by regulation of dendritic cell dendrite assembly [GO:2000547]; RO_0002212 by negative regulation of dendritic cell dendrite assembly [GO:2000548]; RO_0002213 by positive regulation of dendritic cell dendrite assembly [GO:2000549] Note: Note that dendrites of dendritic cells should not be confused with neuronal cell dendrites, which process electrical signals. References: PMID:12200351 Sources: CL:0000451, GOC:BHF